{
  "gene_symbol": "ASCL4",
  "gene": "UniProtKB:Q6XD76",
  "gene_name": "Achaete-scute homolog 4",
  "term_id": "GO:0000981",
  "term_label": "DNA-binding transcription factor activity, RNA polymerase II-specific"
}